{
  "gene": "UniProtKB:P43235",
  "term_label": "extracellular space",
  "term_id": "GO:0005615",
  "gene_name": "Cathepsin K",
  "gene_symbol": "CTSK"
}